{
  "term_label": "nuclear receptor binding",
  "gene": "UniProtKB:Q969G3",
  "gene_symbol": "SMARCE1",
  "term_id": "GO:0016922",
  "gene_name": "SWI_SNF-related matrix-associated actin-dependent regulator of chromatin subfamily E member 1"
}